negative regulation of positive chemotaxis to cAMP by chlorinated alkylphenone [GO:0061125] (biological process) Subtypes: GO:0061127, negative regulation of positive chemotaxis to cAMP by DIF-2 [GO:0061129] Relationships: is a type of regulation of positive chemotaxis to cAMP by chlorinated alkylphenone [GO:0061119]; is a type of negative regulation of positive chemotaxis to cAMP [GO:0061123] Sources: GOC:dph Definition: Any process that decreases the rate, frequency, or extent of directed movement of a motile cell or organism up a concentration gradient of 3',5'-cAMP by the action of a chlorinated alkylphenone. An alkylphenone is an aromatic polyketide with methyl and chlorine substitutions.